positive regulation of embryo sac egg cell differentiation [GO:0045696] (biological process) Definition: Any process that activates or increases the frequency, rate or extent of embryo sac egg cell differentiation. Sources: GOC:go_curators, GOC:mtg_plant Relationships: is a type of positive regulation of cell differentiation [GO:0045597]; is a type of GO:0045694; is a type of positive regulation of multicellular organismal process [GO:0051240]; is a type of GO:2000243; positively regulates embryo sac egg cell differentiation [GO:0009560] Also known as: positive regulation of female gametophyte egg cell differentiation, up regulation of female gametophyte egg cell differentiation, up-regulation of female gametophyte egg cell differentiation, upregulation of female gametophyte egg cell differentiation, activation of female gametophyte egg cell differentiation, stimulation of female gametophyte egg cell differentiation